{
  "gene_symbol": "OR10D3",
  "gene": "UniProtKB:Q8NH80",
  "term_label": "olfactory receptor activity",
  "term_id": "GO:0004984",
  "gene_name": "Olfactory receptor 10D3"
}